{
  "term_id": "GO:0043022",
  "gene_name": "Elongation factor-like GTPase 1",
  "term_label": "ribosome binding",
  "gene_symbol": "EFL1",
  "gene": "UniProtKB:Q7Z2Z2"
}